{
  "gene_name": "Contactin associated protein family member 3C (Fragment)",
  "gene_symbol": "CNTNAP3C",
  "gene": "UniProtKB:A0A1B0GTE1",
  "term_id": "UNKNOWN:0003",
  "term_label": "Unknown cellular component"
}